regulation of zygospore formation [GO:0075298] (biological process) Definition: Any process that modulates the frequency, rate or extent of zygospore formation, a process in which a thick-walled spore of some algae and fungi is formed by union of two similar sexual cells, usually serves as a resting spore, and produces the sporophytic phase. Relationships: is a type of regulation of sexual sporulation resulting in formation of a cellular spore [GO:0043940]; regulates zygospore formation [GO:0034296] Subtypes: GO:0075299, negative regulation of zygospore formation [GO:0075300] Sources: GOC:pamgo_curators